{
  "term_id": "GO:0005634",
  "term_label": "nucleus",
  "gene_name": "Poly [ADP-ribose] polymerase tankyrase-2",
  "gene_symbol": "TNKS2",
  "gene": "UniProtKB:Q9H2K2"
}